regulation of pro-T cell differentiation [GO:2000174] (biological process) Subtypes: GO:2000175, positive regulation of pro-T cell differentiation [GO:2000176] Also known as: regulation of pro-T lymphocyte differentiation Definition: Any process that modulates the frequency, rate or extent of pro-T cell differentiation. Relationships: is_a regulation of T cell differentiation [GO:0045580]; is a type of GO:1905456; RO_0002211 pro-T cell differentiation [GO:0002572] Sources: GOC:BHF